cinnamic acid biosynthetic process [GO:0009800] (biological process) Definition: The chemical reactions and pathways resulting in the formation of cinnamic acid, 3-phenyl-2-propenoic acid. Sources: GOC:jl Also known as: cinnamic acid anabolism, cinnamic acid biosynthesis, cinnamic acid formation, cinnamic acid synthesis, cinnamylic acid biosynthesis, cinnamylic acid biosynthetic process, phenylacrylic acid biosynthesis, phenylacrylic acid biosynthetic process, phenylpropenoic acid biosynthesis, phenylpropenoic acid biosynthetic process Relationships: is a type of phenylpropanoid biosynthetic process [GO:0009699]; is a type of GO:0009803; is a type of monocarboxylic acid biosynthetic process [GO:0072330]; is a type of olefinic compound biosynthetic process [GO:0120255]